{
  "gene": "UniProtKB:Q6PI25",
  "term_label": "synaptic transmission, glutamatergic",
  "gene_name": "Protein cornichon homolog 2",
  "term_id": "GO:0035249",
  "gene_symbol": "CNIH2"
}